{
  "gene_name": "Piercer of microtubule wall 1 protein",
  "gene_symbol": "PIERCE1",
  "term_id": "UNKNOWN:0001",
  "gene": "UniProtKB:Q5BN46",
  "term_label": "Unknown molecular function"
}